{
  "gene": "UniProtKB:Q9H7P9",
  "gene_name": "Pleckstrin homology domain-containing family G member 2",
  "term_label": "guanyl-nucleotide exchange factor activity",
  "gene_symbol": "PLEKHG2",
  "term_id": "GO:0005085"
}